protein-glutamic acid ligase activity, elongating [GO:0106438] (molecular function) Definition: Catalytic reaction :(L-glutamyl)n-L-gamma-glutamyl-L-glutamyl-[protein] + ATP + L-glutamate = (L-glutamyl)n+1-L-gamma-glutamyl-L-glutamyl-[protein] + ADP + H+ + phosphate. References: PMID:32747782 Sources: RHEA:60148 Relationships: is_a protein-glutamic acid ligase activity [GO:0070739]